endoplasmic reticulum stress-induced pre-emptive quality control [GO:0061857] (biological process) Definition: The response to endoplasimic reticulum stress in which nascent proteins are degraded by attenuation of their translocation into the ER followed by rerouting to the cytosol without cleavage of the signal peptide, and subsequent degradation by the proteasome. Relationships: is_a response to endoplasmic reticulum stress [GO:0034976]; has part proteasome-mediated ubiquitin-dependent protein catabolic process [GO:0043161] Also known as: ER pQC, ER stress-indiced pre-emptive quality control References: PMID:17129784, PMID:26565908